{
  "gene": "UniProtKB:Q8WWZ4",
  "gene_symbol": "ABCA10",
  "term_label": "lipid transporter activity",
  "term_id": "GO:0005319",
  "gene_name": "ATP-binding cassette sub-family A member 10"
}